{
  "gene": "UniProtKB:Q9BTT6",
  "gene_name": "Leucine-rich repeat-containing protein 1",
  "term_label": "Unknown molecular function",
  "term_id": "UNKNOWN:0001",
  "gene_symbol": "LRRC1"
}